{
  "gene_symbol": "HLA-DPA1",
  "term_id": "GO:0023026",
  "term_label": "MHC class II protein complex binding",
  "gene_name": "HLA class II histocompatibility antigen, DP alpha 1 chain",
  "gene": "UniProtKB:P20036"
}